{
  "term_label": "inositol bisphosphate phosphatase activity",
  "gene": "UniProtKB:Q9BT40",
  "term_id": "GO:0016312",
  "gene_name": "Inositol polyphosphate 5-phosphatase K",
  "gene_symbol": "INPP5K"
}